{
  "term_label": "protein serine/threonine kinase activity",
  "gene_name": "Mitogen-activated protein kinase kinase kinase kinase 4",
  "term_id": "GO:0004674",
  "gene_symbol": "MAP4K4",
  "gene": "UniProtKB:O95819"
}